{
  "term_label": "chromatin",
  "gene_name": "Chromodomain-helicase-DNA-binding protein 1",
  "term_id": "GO:0000785",
  "gene": "UniProtKB:O14646",
  "gene_symbol": "CHD1"
}